{
  "term_id": "GO:0031492",
  "gene_symbol": "H1-6",
  "term_label": "nucleosomal DNA binding",
  "gene_name": "Histone H1t",
  "gene": "UniProtKB:P22492"
}